cellular response to sucrose starvation [GO:0043617] (biological process) Relationships: is a type of GO:0009267 Sources: GOC:jl Definition: Any process that results in a change in state or activity of a cell (in terms of movement, secretion, enzyme production, gene expression, etc.) as a result of deprivation of sucrose.